protein-serine epimerase activity [GO:0018365] (molecular function) Also known as: protein-serine racemase activity Sources: EC:5.1.1.16 Relationships: is a type of racemase and epimerase activity, acting on amino acids and derivatives [GO:0016855] Definition: Catalysis of the reaction: (protein)-L-serine = (protein)-D-serine.